{
  "gene_symbol": "SFRP4",
  "gene": "UniProtKB:Q6FHJ7",
  "term_label": "canonical Wnt signaling pathway",
  "term_id": "GO:0060070",
  "gene_name": "Secreted frizzled-related protein 4"
}